{
  "term_id": "GO:0042147",
  "term_label": "retrograde transport, endosome to Golgi",
  "gene_symbol": "PHETA2",
  "gene_name": "Sesquipedalian-2",
  "gene": "UniProtKB:Q6ICB4"
}